cyclohexa-1,5-dienecarbonyl-CoA hydratase activity [GO:0018823] (molecular function) Relationships: is a type of hydro-lyase activity [GO:0016836] Also known as: cyclohex-1,5-diene-1-carbonyl-CoA hydratase activity, 6-hydroxycyclohex-1-enecarbonyl-CoA (cyclohexa-1,5-dienecarbonyl-CoA-forming), cyclohexa-1,5-diene-1-carbonyl-CoA hydratase activity, cyclohexa-1,5-diene-1-carboxyl-CoA hydratase activity, cyclohexa-1,5-dienecarbonyl-CoA hydro-lyase activity, dienoyl-CoA hydratase activity Sources: EC:4.2.1.100, RHEA:21856 Definition: Catalysis of the reaction: cyclohexa-1,5-diene-1-carbonyl-CoA + H2O = 6-hydroxycyclohex-1-enecarbonyl-CoA.